{
  "gene_name": "Ribonuclease P protein subunit p38",
  "gene_symbol": "RPP38",
  "term_label": "ribonuclease P RNA binding",
  "gene": "UniProtKB:P78345",
  "term_id": "GO:0033204"
}